{
  "gene": "UniProtKB:P56159",
  "gene_name": "GDNF family receptor alpha-1",
  "term_id": "GO:0007399",
  "term_label": "nervous system development",
  "gene_symbol": "GFRA1"
}